removal of nonhomologous ends [GO:0000735] (biological process) Relationships: is a type of GO:0006259; has part GO:0004520 Definition: The removal of nonhomologous sequences at the broken 3' single-strand DNA end before DNA repair synthesis can occur. References: PMID:10357855 Subtypes: double-strand break repair via single-strand annealing, removal of nonhomologous ends [GO:0000736]